{
  "term_id": "UNKNOWN:0002",
  "gene_name": "Putative uncharacterized protein encoded by LINC02915",
  "term_label": "Unknown biological process",
  "gene": "UniProtKB:Q8N8G6",
  "gene_symbol": "LINC02915"
}